regulation of body fluid levels [GO:0050878] (biological process) Definition: Any process that modulates the levels of body fluids. Sources: GOC:ai, GOC:dph, GOC:tb Relationships: is a type of regulation of biological quality [GO:0065008] Subtypes: body fluid secretion [GO:0007589], hemostasis [GO:0007599], regulation of urine volume [GO:0035809], regulation of saliva secretion [GO:0046877], multicellular organismal-level water homeostasis [GO:0050891], GO:0070255, GO:0090186, regulation of hemostasis [GO:1900046], regulation of lactation [GO:1903487], regulation of renal water transport [GO:2001151]